nucleate erythrocyte development [GO:0048823] (biological process) Relationships: is_a erythrocyte development [GO:0048821]; is part of nucleate erythrocyte differentiation [GO:0043363] Definition: The process aimed at the progression of a nucleate erythrocyte over time, from initial commitment of the cell to a specific fate, to the fully functional differentiated cell. Sources: GOC:devbiol Also known as: nucleate RBC development, nucleate red blood cell development